action potential [GO:0001508] (BP) Regulation: RO_0002212 by negative regulation of action potential [GO:0045759]; positively regulated by positive regulation of action potential [GO:0045760]; regulated by GO:0097364; regulated by regulation of action potential [GO:0098900] Note: Action potentials typically propagate across excitable membranes. This class covers both action potentials that propagate and those that fail to do so. Subtypes: neuronal action potential [GO:0019228], cardiac muscle cell action potential [GO:0086001], action potential propagation [GO:0098870], action potential initiation [GO:0099610], regulation of skeletal muscle contraction by action potential [GO:0100001] Definition: A process in which membrane potential cycles through a depolarizing spike, triggered in response to depolarization above some threshold, followed by repolarization. This cycle is driven by the flow of ions through various voltage gated channels with different thresholds and ion specificities. Sources: GOC:dph, GOC:go_curators, GOC:tb, ISBN:978-0-07-139011-8 Relationships: is a type of regulation of membrane potential [GO:0042391]